{
  "term_id": "GO:0061631",
  "term_label": "ubiquitin conjugating enzyme activity",
  "gene_name": "Ubiquitin-conjugating enzyme E2 Z",
  "gene": "UniProtKB:Q9H832",
  "gene_symbol": "UBE2Z"
}